G protein-coupled pyrimidinergic nucleotide receptor activity [GO:0071553] (MF) Relationships: is a type of G protein-coupled receptor activity [GO:0004930]; is a type of nucleotide receptor activity [GO:0016502]; has part pyrimidine nucleotide binding [GO:0019103] Definition: Combining with a pyrimidine nucleotide and transmitting the signal across the membrane by activating an associated G-protein; promotes the exchange of GDP for GTP on the alpha subunit of a heterotrimeric G-protein complex. Subtypes: G protein-coupled UDP receptor activity [GO:0045029], G protein-coupled UTP receptor activity [GO:0045030] Also known as: G protein coupled pyrimidinergic nucleotide receptor activity, G-protein coupled pyrimidinergic nucleotide receptor activity, pyrimidinergic nucleotide receptor activity, G protein coupled, pyrimidinergic nucleotide receptor activity, G-protein coupled References: PMID:10736418, PMID:12369950, PMID:15796906 Sources: GOC:sl